{
  "term_label": "heterochromatin formation",
  "gene_name": "Histone H3.3",
  "gene": "UniProtKB:P84243",
  "gene_symbol": "H3-3B",
  "term_id": "GO:0031507"
}